chlorophyll a biosynthetic process via geranylgeranyl-chlorophyll a [GO:0033312] (biological process) Definition: The chemical reactions and pathways leading to the formation of chlorophyll a, via the intermediate geranylgeranyl-chlorophyll a. Sources: GOC:mah, MetaCyc:PWY-5064 Also known as: chlorophyll a anabolism via geranylgeranyl-chlorophyll a, chlorophyll a biosynthesis via geranylgeranyl-chlorophyll a, chlorophyll a formation via geranylgeranyl-chlorophyll a, chlorophyll a synthesis via geranylgeranyl-chlorophyll a Relationships: is a type of chlorophyll a biosynthetic process [GO:0033305]